upstream stimulatory factor complex [GO:1990378] (cellular component) Also known as: USF complex, USF1 homodimer, USF1-USF2 heterodimer, USF2 homodimer Definition: A protein complex capable of sequence-specific DNA binding RNA polymerase II transcription factor activity through binding to a symmetrical DNA sequence (E-boxes) (5'-CACGTG-3'). Found in a variety of viral and cellular promoters. Note: An example of this is USF1 in human (UniProt symbol P22415) in PMID:8576131 (inferred from direct assay). Relationships: is a type of RNA polymerase II transcription regulator complex [GO:0090575] References: PMID:8576131 Sources: GOC:bhm